{
  "gene_name": "Interferon regulatory factor 2",
  "term_id": "GO:0000978",
  "gene_symbol": "IRF2",
  "gene": "UniProtKB:P14316",
  "term_label": "RNA polymerase II cis-regulatory region sequence-specific DNA binding"
}